negative regulation of response to macrophage colony-stimulating factor [GO:1903970] (biological process) Also known as: down regulation of response to M-CSF, down regulation of response to macrophage colony-stimulating factor, down regulation of response to macrophage colony-stimulating factor stimulus, down-regulation of response to M-CSF, down-regulation of response to macrophage colony-stimulating factor, down-regulation of response to macrophage colony-stimulating factor stimulus, downregulation of response to M-CSF, downregulation of response to macrophage colony-stimulating factor, downregulation of response to macrophage colony-stimulating factor stimulus, negative regulation of response to M-CSF, negative regulation of response to macrophage colony-stimulating factor stimulus, inhibition of response to M-CSF, inhibition of response to macrophage colony-stimulating factor, inhibition of response to macrophage colony-stimulating factor stimulus References: PMID:19100238 Sources: GOC:BHF, GOC:TermGenie, GOC:nc, GO_REF:0000058 Relationships: is a type of GO:0060761; is a type of regulation of response to macrophage colony-stimulating factor [GO:1903969]; negatively regulates GO:0036005 Subtypes: negative regulation of cellular response to macrophage colony-stimulating factor stimulus [GO:1903973] Definition: Any process that stops, prevents or reduces the frequency, rate or extent of response to macrophage colony-stimulating factor.